{
  "gene": "UniProtKB:P05556",
  "term_label": "fibronectin binding",
  "gene_name": "Integrin beta-1",
  "gene_symbol": "ITGB1",
  "term_id": "GO:0001968"
}